3-alpha,7-alpha-dihydroxy-5-beta-cholestanate-CoA ligase activity [GO:0047476] (molecular function) Relationships: is a type of CoA-ligase activity [GO:0016405]; is a type of acid-thiol ligase activity [GO:0016878] Also known as: 3alpha,7alpha-dihydroxy-5beta-cholestanate-CoA ligase activity, 3alpha,7alpha-dihydroxy-5beta-cholestanate:CoA ligase (AMP-forming), 3alpha,7alpha-dihydroxy-5beta-cholestanoyl coenzyme A synthetase activity, DHCA-CoA ligase activity Definition: Catalysis of the reaction: CoA + 3-alpha,7-alpha-dihydroxy-5-beta-cholestanate + ATP = 3-alpha,7-alpha-dihydroxy-5-beta-cholestanoyl-CoA + diphosphate + AMP. Sources: EC:6.2.1.28, MetaCyc:6.2.1.28-RXN